{
  "gene_name": "Phosducin-like protein",
  "term_label": "cytoplasm",
  "gene_symbol": "PDCL",
  "term_id": "GO:0005737",
  "gene": "UniProtKB:Q13371"
}